maintenance of protein location in extracellular region [GO:0071694] (biological process) Sources: GOC:mah Definition: Any process in which a protein is maintained in a specific location within the extracellular region and is prevented from moving elsewhere. Subtypes: sequestering of BMP in extracellular matrix [GO:0035582], sequestering of TGFbeta in extracellular matrix [GO:0035583] Relationships: is a type of maintenance of protein location [GO:0045185]; is part of GO:0071692